6-beta-hydroxyhyoscyamine epoxidase activity [GO:0047594] (molecular function) Sources: EC:1.14.20.13, RHEA:12797 Relationships: is a type of 2-oxoglutarate-dependent dioxygenase activity [GO:0016706] Definition: Catalysis of the reaction: (6S)-6-hydroxyhyoscyamine + 2-oxoglutarate + O2 = CO2 + H2O + H+ + scopolamine + succinate. Also known as: (6S)-6-hydroxyhyoscyamine,2-oxoglutarate oxidoreductase (epoxide-forming), 6beta-hydroxyhyoscyamine epoxidase activity, hydroxyhyoscyamine dioxygenase activity